detection of chemical stimulus involved in sensory perception of smell [GO:0050911] (biological process) Sources: GOC:ai Definition: The series of events involved in the perception of smell in which an olfactory chemical stimulus is received and converted into a molecular signal. Relationships: is_a detection of chemical stimulus involved in sensory perception [GO:0050907]; is part of sensory perception of smell [GO:0007608] Also known as: perception of smell, detection of chemical stimulus, perception of smell, sensory detection of chemical stimulus, perception of smell, sensory transduction of chemical stimulus, sensory detection of chemical stimulus during perception of smell, sensory detection of scent, sensory detection of smell, sensory transduction of chemical stimulus during perception of smell, sensory transduction of scent, sensory transduction of smell